{
  "term_label": "sperm flagellum assembly",
  "gene_name": "Cilia- and flagella-associated protein 61",
  "term_id": "GO:0120316",
  "gene_symbol": "CFAP61",
  "gene": "UniProtKB:Q8NHU2"
}